O-acyl-L-carnitine transmembrane transporter activity [GO:0015227] (molecular function) Subtypes: carnitine:O-acyl-L-carnitine antiporter activity [GO:0005476] Sources: GOC:ai Also known as: acylcarnitine transporter activity Relationships: is a type of quaternary ammonium group transmembrane transporter activity [GO:0015651]; is part of GO:1902616 Definition: Enables the transfer of O-acyl-L-carnitine from one side of a membrane to the other. O-acyl-L-carnitine is the condensation product of a carboxylic acid and carnitine and is the transport form for a fatty acid crossing the mitochondrial membrane.